{
  "term_id": "GO:0000956",
  "term_label": "nuclear-transcribed mRNA catabolic process",
  "gene_symbol": "POLR2G",
  "gene": "UniProtKB:P62487",
  "gene_name": "DNA-directed RNA polymerase II subunit RPB7"
}